translation regulator activity [GO:0045182] (molecular function) Definition: Any molecular function involved in the regulation of initiation, activation, perpetuation, repression or termination of polypeptide synthesis at the ribosome. Sources: GOC:ai Relationships: is a type of GO:0003674; is part of GO:0006417 Subtypes: translation activator activity [GO:0008494], translation repressor activity [GO:0030371]